{
  "term_label": "proteasome-mediated ubiquitin-dependent protein catabolic process",
  "gene_symbol": "UBE2B",
  "gene": "UniProtKB:P63146",
  "gene_name": "Ubiquitin-conjugating enzyme E2 B",
  "term_id": "GO:0043161"
}